intracellular canaliculus [GO:0046691] (CC) Also known as: canalicular membrane References: PMID:10700045 Sources: GOC:mah, ISBN:0721662544 Definition: An apical plasma membrane part that forms a narrow enfolded luminal membrane channel, lined with numerous microvilli, that appears to extend into the cytoplasm of the cell. A specialized network of intracellular canaliculi is a characteristic feature of parietal cells of the gastric mucosa in vertebrates. Relationships: is a type of cellular anatomical structure [GO:0110165]; is part of GO:0016324